{
  "term_id": "UNKNOWN:0002",
  "gene_symbol": "RALYL",
  "term_label": "Unknown biological process",
  "gene_name": "RNA-binding Raly-like protein",
  "gene": "UniProtKB:Q86SE5"
}